{
  "gene": "UniProtKB:Q15004",
  "term_id": "GO:0003682",
  "gene_symbol": "PCLAF",
  "gene_name": "PCNA-associated factor",
  "term_label": "chromatin binding"
}